{
  "term_label": "Unknown biological process",
  "gene": "UniProtKB:Q5TA77",
  "term_id": "UNKNOWN:0002",
  "gene_name": "Late cornified envelope protein 3B",
  "gene_symbol": "LCE3B"
}